negative extrathymic T cell selection [GO:0045068] (biological process) References: PMID:7880383 Sources: ISBN:0781735149 Also known as: negative extrathymic T lymphocyte selection, negative extrathymic T-cell selection, negative extrathymic T-lymphocyte selection Definition: The process of elimination of extrathymically maturing T cells which react strongly with self-antigens. Relationships: is a type of GO:0043383; is a type of extrathymic T cell selection [GO:0045062]